dADP metabolic process [GO:0046056] (biological process) Definition: The chemical reactions and pathways involving dADP, deoxyadenosine diphosphate (2'-deoxyadenosine 5'-diphosphate). Subtypes: dADP biosynthetic process [GO:0006173], dADP catabolic process [GO:0046057] Relationships: is a type of GO:0009151; is a type of purine deoxyribonucleoside diphosphate metabolic process [GO:0009182] Sources: GOC:go_curators Also known as: dADP metabolism